{
  "gene_name": "G-protein coupled receptor 42",
  "gene": "UniProtKB:O15529",
  "term_id": "GO:0005886",
  "term_label": "plasma membrane",
  "gene_symbol": "GPR42"
}